{
  "gene_name": "RING finger protein 208",
  "gene": "UniProtKB:Q9H0X6",
  "term_label": "ubiquitin protein ligase activity",
  "term_id": "GO:0061630",
  "gene_symbol": "RNF208"
}